{
  "gene_symbol": "SLC46A3",
  "gene_name": "Lysosomal proton-coupled steroid conjugate and bile acid symporter SLC46A3",
  "gene": "UniProtKB:Q7Z3Q1",
  "term_id": "GO:0005765",
  "term_label": "lysosomal membrane"
}